{
  "term_id": "GO:0003777",
  "gene_symbol": "KIF13B",
  "gene": "UniProtKB:Q9NQT8",
  "term_label": "microtubule motor activity",
  "gene_name": "Kinesin-like protein KIF13B"
}